{
  "gene_name": "Cyclic nucleotide-gated cation channel alpha-3",
  "gene_symbol": "CNGA3",
  "term_label": "intracellularly cGMP-activated cation channel activity",
  "gene": "UniProtKB:Q16281",
  "term_id": "GO:0005223"
}